{
  "term_label": "double-strand break repair via homologous recombination",
  "gene_name": "Serine_threonine-protein phosphatase 4 catalytic subunit",
  "gene_symbol": "PPP4C",
  "gene": "UniProtKB:P60510",
  "term_id": "GO:0000724"
}